{
  "gene_symbol": "GPT",
  "gene_name": "Alanine aminotransferase 1",
  "term_label": "Unknown molecular function",
  "gene": "UniProtKB:P24298",
  "term_id": "UNKNOWN:0001"
}